chemokine receptor binding [GO:0042379] (molecular function) Relationships: is a type of G protein-coupled receptor binding [GO:0001664]; is a type of cytokine receptor binding [GO:0005126] Also known as: chemokine receptor ligand Definition: Binding to a chemokine receptor. Subtypes: chemokine activity [GO:0008009], GO:0031737, XCR1 chemokine receptor binding [GO:0031738], CXCR chemokine receptor binding [GO:0045236], GO:0048020 Sources: GOC:ai